{
  "term_id": "UNKNOWN:0002",
  "gene_symbol": "PTPN4",
  "gene": "UniProtKB:P29074",
  "gene_name": "Tyrosine-protein phosphatase non-receptor type 4",
  "term_label": "Unknown biological process"
}